DNA replication factor C core complex [GO:0070517] (cellular component) References: PMID:8692848, PMID:9228079, PMID:9582326 Also known as: RFC core complex Relationships: is a type of nuclear protein-containing complex [GO:0140513]; BFO_0000050 GO:0043599 Definition: A protein complex containing three of the five subunits of eukaryotic replication factor C, those corresponding to human p40, p38, and p37.